R8 cell development [GO:0045463] (biological process) References: PMID:11880339 Definition: The process whose specific outcome is the progression of the R8 photoreceptor over time, from its formation to the mature structure. The R8 photoreceptor is the founding receptor of each ommatidium. Relationships: is a type of compound eye photoreceptor development [GO:0042051]; is part of GO:0045465